{
  "gene": "UniProtKB:Q96LT9",
  "gene_symbol": "RNPC3",
  "term_label": "pre-mRNA intronic binding",
  "gene_name": "RNA-binding region-containing protein 3",
  "term_id": "GO:0097157"
}